{
  "term_id": "GO:0005856",
  "gene_symbol": "KRT34",
  "gene_name": "Keratin, type I cuticular Ha4",
  "term_label": "cytoskeleton",
  "gene": "UniProtKB:O76011"
}